{
  "term_id": "UNKNOWN:0003",
  "gene_name": "Zinc finger protein 366",
  "gene": "UniProtKB:Q8N895",
  "gene_symbol": "ZNF366",
  "term_label": "Unknown cellular component"
}